{
  "term_label": "glutamatergic synapse",
  "gene_name": "Cerebellin-1",
  "gene": "UniProtKB:P23435",
  "gene_symbol": "CBLN1",
  "term_id": "GO:0098978"
}